{
  "gene_symbol": "TLDC2",
  "term_id": "UNKNOWN:0001",
  "gene_name": "TLD domain-containing protein 2",
  "gene": "UniProtKB:A0PJX2",
  "term_label": "Unknown molecular function"
}